H-NS-Cnu complex [GO:0036411] (cellular component) References: PMID:18189420, PMID:22358512 Sources: GOC:bhm Definition: A trimeric protein complex containing a H-NS homodimer and a Cnu monomer. In bacteria, this complex negatively regulates transcription of a range of genes. Relationships: is a type of transcription repressor complex [GO:0017053]; has part H-NS complex [GO:1990121]